regulation of monocyte differentiation [GO:0045655] (biological process) Subtypes: negative regulation of monocyte differentiation [GO:0045656], positive regulation of monocyte differentiation [GO:0045657] Relationships: is a type of regulation of myeloid leukocyte differentiation [GO:0002761]; regulates monocyte differentiation [GO:0030224] Definition: Any process that modulates the frequency, rate or extent of monocyte differentiation. Sources: GOC:go_curators